{
  "gene_name": "Histone deacetylase complex subunit SAP25",
  "term_label": "Unknown cellular component",
  "gene": "UniProtKB:Q8TEE9",
  "gene_symbol": "SAP25",
  "term_id": "UNKNOWN:0003"
}